{
  "gene": "UniProtKB:Q86UD7",
  "gene_symbol": "TBC1D26",
  "term_label": "Unknown cellular component",
  "term_id": "UNKNOWN:0003",
  "gene_name": "TBC1 domain family member 26"
}